{
  "term_label": "cytosol",
  "term_id": "GO:0005829",
  "gene_symbol": "PPM1F",
  "gene_name": "Protein phosphatase 1F",
  "gene": "UniProtKB:P49593"
}